tubulin-glycine ligase activity [GO:0070738] (molecular function) References: PMID:19524510 Sources: GOC:mah Relationships: is a type of protein-glycine ligase activity [GO:0070735] Definition: Catalysis of the posttranslational transfer of one or more glycine residues to a specific glutamate residue on a target tubulin molecule; acts on alpha or beta tubulin. Also known as: tubulin glycylase activity